pseudophosphatase activity [GO:0001691] (molecular function) Definition: Maintains the phosphorylation state of certain molecules by associating with them and preventing them from associating with active phosphatases, and thus inhibiting the enzyme activity without interacting with the enzyme. Often pertains to proteins belonging to dual-specificity phosphatase family but lacking critical active site residues. Sources: GOC:ajp Relationships: is a type of phosphatase inhibitor activity [GO:0019212]